{
  "gene": "UniProtKB:Q96P15",
  "term_label": "extracellular space",
  "gene_symbol": "SERPINB11",
  "term_id": "GO:0005615",
  "gene_name": "Serpin B11"
}